{
  "term_id": "GO:0009328",
  "term_label": "phenylalanine-tRNA ligase complex",
  "gene_name": "Phenylalanine--tRNA ligase alpha subunit",
  "gene_symbol": "FARSA",
  "gene": "UniProtKB:Q9Y285"
}